{
  "gene_symbol": "BIRC2",
  "gene_name": "Baculoviral IAP repeat-containing protein 2",
  "gene": "UniProtKB:Q13490",
  "term_label": "negative regulation of necroptotic process",
  "term_id": "GO:0060546"
}